beta-catenin destruction complex disassembly [GO:1904886] (biological process) Definition: The disaggregation of a beta-catenin destruction complex into its constituent components. Relationships: is a type of protein-containing complex disassembly [GO:0032984]; is part of canonical Wnt signaling pathway [GO:0060070] Also known as: APC-Axin-1-beta-catenin complex disassembly, Axin-APC-beta-catenin-GSK3B complex disassembly, BDC disassembly, beta-catenin degradation complex disassembly, dissociation of beta-catenin degradation complex, 23S APC complex disassembly References: PMID:23169527 Sources: GOC:PARL, GOC:TermGenie, GOC:bf, GO_REF:0000079